{
  "gene_name": "Ubiquitin-protein ligase E3B",
  "gene": "UniProtKB:Q7Z3V4",
  "term_label": "protein polyubiquitination",
  "gene_symbol": "UBE3B",
  "term_id": "GO:0000209"
}